{
  "gene_symbol": "GJB2",
  "gene": "UniProtKB:P29033",
  "term_label": "inner ear development",
  "gene_name": "Gap junction beta-2 protein",
  "term_id": "GO:0048839"
}